{
  "term_id": "UNKNOWN:0003",
  "term_label": "Unknown cellular component",
  "gene_name": "Integrator complex subunit 14",
  "gene": "UniProtKB:Q96SY0",
  "gene_symbol": "INTS14"
}